{
  "term_label": "Unknown cellular component",
  "term_id": "UNKNOWN:0003",
  "gene_symbol": "CCDC93",
  "gene": "UniProtKB:Q567U6",
  "gene_name": "Coiled-coil domain-containing protein 93"
}